pigment accumulation [GO:0043476] (biological process) Subtypes: pigment accumulation in response to UV light [GO:0043478], pigment accumulation in tissues [GO:0043480], GO:0043482, melanization of appressorium wall [GO:0075043] Sources: GOC:jl Also known as: pigment accumulation in response to external stimulus Relationships: is a type of response to external stimulus [GO:0009605]; is a type of GO:0043473 Definition: The aggregation of coloring matter in a particular location in an organism, tissue or cell, occurring in response to some external stimulus.